mevalonate transmembrane transporter activity [GO:0015130] (molecular function) Definition: Enables the transfer of mevalonate from one side of a membrane to the other. Mevalonate is the anion of mevalonic acid; its (R)-enantiomer is a strategic intermediate derived from hydroxymethylglutaryl-CoA in the biosynthesis of polyprenyl compounds. Sources: GOC:ai, ISBN:0198506732 Also known as: monocarboxylate (lactate, pyruvate, mevalonate) uptake/efflux porter activity Relationships: is a type of GO:0022857; is part of GO:0015728